{
  "gene_symbol": "ADAM33",
  "term_label": "metalloendopeptidase activity",
  "gene_name": "Disintegrin and metalloproteinase domain-containing protein 33",
  "gene": "UniProtKB:Q9BZ11",
  "term_id": "GO:0004222"
}